{
  "term_id": "UNKNOWN:0003",
  "gene_name": "Stromal cell-derived factor 2-like protein 1",
  "gene_symbol": "SDF2L1",
  "gene": "UniProtKB:Q9HCN8",
  "term_label": "Unknown cellular component"
}